{
  "gene_name": "Claudin-2",
  "term_label": "plasma membrane",
  "gene_symbol": "CLDN2",
  "term_id": "GO:0005886",
  "gene": "UniProtKB:P57739"
}